cellular response to hydroperoxide [GO:0071447] (biological process) Relationships: is a type of response to hydroperoxide [GO:0033194]; is a type of cellular response to oxidative stress [GO:0034599]; is a type of cellular response to oxygen-containing compound [GO:1901701] Sources: GOC:mah Subtypes: cellular response to alkyl hydroperoxide [GO:0071448], cellular response to lipid hydroperoxide [GO:0071449] Definition: Any process that results in a change in state or activity of a cell (in terms of movement, secretion, enzyme production, gene expression, etc.) as a result of a hydroperoxide stimulus. Hydroperoxides are monosubstitution products of hydrogen peroxide, HOOH.